{
  "term_id": "GO:0006357",
  "gene_symbol": "ZNF541",
  "term_label": "regulation of transcription by RNA polymerase II",
  "gene": "UniProtKB:Q9H0D2",
  "gene_name": "Zinc finger protein 541"
}